{
  "term_id": "GO:0000122",
  "gene_symbol": "MAGEA10",
  "gene": "UniProtKB:P43363",
  "term_label": "negative regulation of transcription by RNA polymerase II",
  "gene_name": "Melanoma-associated antigen 10"
}